{
  "gene_name": "Transcription elongation factor A protein-like 6",
  "gene_symbol": "TCEAL6",
  "term_label": "Unknown molecular function",
  "gene": "UniProtKB:Q6IPX3",
  "term_id": "UNKNOWN:0001"
}